{
  "gene_symbol": "IGFL4",
  "gene": "UniProtKB:Q6B9Z1",
  "term_label": "signaling receptor binding",
  "gene_name": "Insulin growth factor-like family member 4",
  "term_id": "GO:0005102"
}